positive regulation of epithelial tube formation [GO:1905278] (biological process) Note: An example of this is MMRN2 in human (Q9H8L6) in PMID:25745997 (inferred from direct assay). References: PMID:25745997 Sources: GOC:TermGenie, GOC:bhm, GO_REF:0000058 Relationships: is a type of positive regulation of multicellular organismal process [GO:0051240]; is a type of regulation of epithelial tube formation [GO:1905276]; is a type of positive regulation of morphogenesis of an epithelium [GO:1905332]; positively regulates epithelial tube formation [GO:0072175] Definition: Any process that activates or increases the frequency, rate or extent of epithelial tube formation. Subtypes: pancreas induction [GO:0061132], positive regulation of ureteric bud formation [GO:0072107] Also known as: up regulation of epithelial tube formation, up-regulation of epithelial tube formation, upregulation of epithelial tube formation, activation of epithelial tube formation